{
  "term_id": "GO:0005737",
  "gene_name": "Myotubularin-related protein 13",
  "term_label": "cytoplasm",
  "gene_symbol": "SBF2",
  "gene": "UniProtKB:Q86WG5"
}